{
  "term_label": "cytosol",
  "gene_symbol": "ARHGEF10L",
  "gene_name": "Rho guanine nucleotide exchange factor 10-like protein",
  "term_id": "GO:0005829",
  "gene": "UniProtKB:Q9HCE6"
}